response to staurosporine [GO:0072733] (BP) Relationships: is a type of response to alkaloid [GO:0043279] Subtypes: cellular response to staurosporine [GO:0072734] Sources: GOC:mah Definition: Any process that results in a change in state or activity of a cell or an organism (in terms of movement, secretion, enzyme production, gene expression, etc.) as a result of a staurosporine stimulus.